acetylindoxyl oxidase activity [GO:0047608] (molecular function) Sources: EC:1.7.3.2 Definition: Catalysis of the reaction: N-acetylindoxyl + O2 = N-acetylisatin + unknown. Also known as: N-acetylindoxyl:oxygen oxidoreductase activity Relationships: is a type of oxidoreductase activity, acting on other nitrogenous compounds as donors, oxygen as acceptor [GO:0016663]